{
  "gene": "UniProtKB:O15118",
  "term_id": "GO:0015485",
  "gene_symbol": "NPC1",
  "term_label": "cholesterol binding",
  "gene_name": "NPC intracellular cholesterol transporter 1"
}